{
  "term_id": "UNKNOWN:0001",
  "gene_name": "Protein FAM219A",
  "gene_symbol": "FAM219A",
  "term_label": "Unknown molecular function",
  "gene": "UniProtKB:Q8IW50"
}